{
  "gene_symbol": "HNRNPR",
  "term_label": "mRNA binding",
  "term_id": "GO:0003729",
  "gene_name": "Heterogeneous nuclear ribonucleoprotein R",
  "gene": "UniProtKB:O43390"
}